{
  "term_label": "complement activation",
  "gene_name": "Complement C4-B",
  "term_id": "GO:0006956",
  "gene": "UniProtKB:P0C0L5",
  "gene_symbol": "C4B_2"
}